{
  "term_label": "Unknown molecular function",
  "gene_symbol": "TMEM80",
  "term_id": "UNKNOWN:0001",
  "gene": "UniProtKB:Q96HE8",
  "gene_name": "Transmembrane protein 80"
}